{
  "gene": "UniProtKB:P27701",
  "term_label": "Unknown biological process",
  "gene_name": "CD82 antigen",
  "term_id": "UNKNOWN:0002",
  "gene_symbol": "CD82"
}